{
  "gene_name": "Ly6_PLAUR domain-containing protein 6",
  "term_label": "Unknown cellular component",
  "gene": "UniProtKB:Q86Y78",
  "gene_symbol": "LYPD6",
  "term_id": "UNKNOWN:0003"
}